detection of muscle stretch [GO:0035995] (biological process) References: PMID:14583192 Relationships: is a type of response to muscle stretch [GO:0035994]; is a type of detection of mechanical stimulus [GO:0050982] Definition: The series of events by which a muscle stretch stimulus is received by a cell and converted into a molecular signal.